{
  "gene_name": "Scinderin",
  "term_id": "GO:0015629",
  "gene": "UniProtKB:Q9Y6U3",
  "term_label": "actin cytoskeleton",
  "gene_symbol": "SCIN"
}